{
  "gene": "UniProtKB:Q5SGD2",
  "gene_symbol": "PPM1L",
  "gene_name": "Protein phosphatase 1L",
  "term_id": "GO:0007165",
  "term_label": "signal transduction"
}